endocardium morphogenesis [GO:0003160] (biological process) Relationships: is a type of GO:0009653; BFO_0000050 endocardium development [GO:0003157] Definition: The process in which the anatomical structure of the endocardium is generated and organized. The endocardium is an anatomical structure comprised of an endothelium and an extracellular matrix that forms the innermost layer of tissue of the heart, and lines the heart chambers. Sources: GOC:mtg_heart